{
  "gene_name": "Ubiquitin-like protein ATG12",
  "term_id": "GO:0097352",
  "term_label": "autophagosome maturation",
  "gene": "UniProtKB:O94817",
  "gene_symbol": "ATG12"
}